{
  "gene_symbol": "SHB",
  "gene": "UniProtKB:Q15464",
  "term_label": "Unknown biological process",
  "gene_name": "SH2 domain-containing adapter protein B",
  "term_id": "UNKNOWN:0002"
}